{
  "term_label": "phagophore assembly site membrane",
  "term_id": "GO:0034045",
  "gene_name": "WD repeat domain phosphoinositide-interacting protein 2",
  "gene": "UniProtKB:Q9Y4P8",
  "gene_symbol": "WIPI2"
}